{
  "term_id": "GO:0015886",
  "term_label": "heme transport",
  "gene_name": "ATP-binding cassette sub-family B member 6",
  "gene_symbol": "ABCB6",
  "gene": "UniProtKB:Q9NP58"
}